WW domain binding [GO:0050699] (molecular function) Relationships: is a type of protein domain specific binding [GO:0019904] Definition: Binding to a WW domain of a protein, a small module composed of 40 amino acids and plays a role in mediating protein-protein interactions via proline-rich regions. References: PMID:14531730